{
  "gene_name": "Fibroblast growth factor 6",
  "term_label": "fibroblast growth factor receptor binding",
  "term_id": "GO:0005104",
  "gene": "UniProtKB:P10767",
  "gene_symbol": "FGF6"
}